{
  "gene": "UniProtKB:Q8NEB9",
  "term_label": "endocytosis",
  "gene_name": "Phosphatidylinositol 3-kinase catalytic subunit type 3",
  "gene_symbol": "PIK3C3",
  "term_id": "GO:0006897"
}